{
  "term_id": "GO:0007411",
  "gene_name": "Cell adhesion molecule DSCAML1",
  "gene": "UniProtKB:Q8TD84",
  "term_label": "axon guidance",
  "gene_symbol": "DSCAML1"
}